{
  "gene_name": "Heme oxygenase 1",
  "gene": "UniProtKB:P09601",
  "gene_symbol": "HMOX1",
  "term_label": "heme binding",
  "term_id": "GO:0020037"
}